{
  "term_id": "GO:0004143",
  "gene": "UniProtKB:Q53H12",
  "gene_name": "Acylglycerol kinase, mitochondrial",
  "term_label": "ATP-dependent diacylglycerol kinase activity",
  "gene_symbol": "AGK"
}